{
  "term_id": "UNKNOWN:0002",
  "term_label": "Unknown biological process",
  "gene_name": "Putative serpin A13",
  "gene": "UniProtKB:Q6UXR4",
  "gene_symbol": "SERPINA13P"
}